{
  "gene_symbol": "DDX25",
  "gene_name": "ATP-dependent RNA helicase DDX25",
  "gene": "UniProtKB:Q9UHL0",
  "term_label": "RNA helicase activity",
  "term_id": "GO:0003724"
}